{
  "term_label": "Unknown cellular component",
  "gene_name": "Retinol dehydrogenase 16",
  "gene_symbol": "RDH16",
  "term_id": "UNKNOWN:0003",
  "gene": "UniProtKB:O75452"
}